{
  "term_id": "GO:0005667",
  "gene_name": "LIM domain-binding protein 1",
  "gene_symbol": "LDB1",
  "gene": "UniProtKB:Q86U70",
  "term_label": "transcription regulator complex"
}